{
  "term_label": "DNA-binding transcription factor activity, RNA polymerase II-specific",
  "term_id": "GO:0000981",
  "gene_symbol": "ZSCAN18",
  "gene_name": "Zinc finger and SCAN domain-containing protein 18",
  "gene": "UniProtKB:Q8TBC5"
}